{
  "term_id": "GO:0048179",
  "gene_symbol": "ACVR2B",
  "gene": "UniProtKB:Q13705",
  "term_label": "activin receptor complex",
  "gene_name": "Activin receptor type-2B"
}